gap filling involved in double-strand break repair via nonhomologous end joining [GO:0061674] (biological process) Definition: Repair of the gaps in the DNA helix using a discontinuous template during double-strand break repair via nonhomologous end joining. Relationships: is a type of GO:0006259; is part of double-strand break repair via nonhomologous end joining [GO:0006303] Sources: GOC:dph